{
  "gene_name": "Protein enabled homolog",
  "term_label": "actin polymerization or depolymerization",
  "gene": "UniProtKB:Q8N8S7",
  "gene_symbol": "ENAH",
  "term_id": "GO:0008154"
}